regulation of vascular endothelial growth factor receptor signaling pathway [GO:0030947] (biological process) Definition: Any process that modulates the frequency, rate or extent of vascular endothelial growth factor receptor signaling pathway activity. Relationships: is a type of GO:0009966; is a type of regulation of cellular response to growth factor stimulus [GO:0090287]; regulates vascular endothelial growth factor receptor signaling pathway [GO:0048010] Subtypes: negative regulation of vascular endothelial growth factor receptor signaling pathway [GO:0030948], positive regulation of vascular endothelial growth factor receptor signaling pathway [GO:0030949] Also known as: regulation of VEGF receptor signaling pathway, regulation of VEGF receptor signalling pathway, regulation of vascular endothelial growth factor receptor signalling pathway Sources: GOC:dgh